cellular response to triglyceride [GO:0071401] (biological process) Sources: GOC:mah Definition: Any process that results in a change in state or activity of a cell (in terms of movement, secretion, enzyme production, gene expression, etc.) as a result of a triglyceride stimulus. Also known as: cellular response to triacylglyceride, cellular response to triacylglycerol Relationships: is a type of GO:0034014; is a type of cellular response to lipid [GO:0071396]; is a type of cellular response to oxygen-containing compound [GO:1901701]